{
  "term_label": "cytoplasm",
  "gene_symbol": "RBPMS2",
  "gene_name": "RNA-binding protein with multiple splicing 2",
  "term_id": "GO:0005737",
  "gene": "UniProtKB:Q6ZRY4"
}